{
  "gene": "UniProtKB:P30550",
  "gene_name": "Gastrin-releasing peptide receptor",
  "term_id": "GO:0007186",
  "gene_symbol": "GRPR",
  "term_label": "G protein-coupled receptor signaling pathway"
}